{
  "gene": "UniProtKB:Q9H0K1",
  "term_label": "intracellular signal transduction",
  "gene_symbol": "SIK2",
  "term_id": "GO:0035556",
  "gene_name": "Serine_threonine-protein kinase SIK2"
}